regulation of glucose catabolic process to lactate via pyruvate [GO:1904023] (biological process) Definition: Any process that modulates the frequency, rate or extent of glucose catabolic process to lactate via pyruvate. References: PMID:20935145 Sources: GOC:TermGenie, GOC:dph, GO_REF:0000058 Subtypes: negative regulation of glucose catabolic process to lactate via pyruvate [GO:1904024], GO:1904025 Relationships: is_a regulation of glucose metabolic process [GO:0010906]; is a type of regulation of fermentation [GO:0043465]; is a type of regulation of carbohydrate catabolic process [GO:0043470]; regulates GO:0019661 Also known as: regulation of glucose fermentation to lactate via pyruvate, regulation of homofermentation, regulation of homofermentative lactate fermentation, regulation of homofermentative pathway, regulation of homolactate fermentation, regulation of homolactic fermentation